{
  "gene": "UniProtKB:Q9Y3B9",
  "gene_symbol": "RRP15",
  "term_id": "GO:0000470",
  "term_label": "maturation of LSU-rRNA",
  "gene_name": "RRP15-like protein"
}